{
  "term_label": "Unknown cellular component",
  "gene_symbol": "CCDC140",
  "term_id": "UNKNOWN:0003",
  "gene_name": "Coiled-coil domain-containing protein 140",
  "gene": "UniProtKB:Q96MF4"
}